{
  "gene_name": "Olfactory receptor 4F21",
  "term_id": "UNKNOWN:0002",
  "gene_symbol": "OR4F21",
  "gene": "UniProtKB:O95013",
  "term_label": "Unknown biological process"
}